{
  "gene_symbol": "MED4",
  "term_id": "GO:0003712",
  "term_label": "transcription coregulator activity",
  "gene": "UniProtKB:Q9NPJ6",
  "gene_name": "Mediator of RNA polymerase II transcription subunit 4"
}